prostate gland stromal morphogenesis [GO:0060741] (biological process) Definition: The process in which the prostate gland stroma is generated and organized. The prostate gland stroma is made up of the mesenchymal or fibroblast cells of the prostate gland. Sources: GOC:dph Relationships: is a type of developmental process involved in reproduction [GO:0003006]; is a type of GO:0009653; is part of prostate gland morphogenesis [GO:0060512]; is part of connective tissue development [GO:0061448]